collagen type III trimer [GO:0005586] (cellular component) References: PMID:21421911 Definition: A collagen homotrimer of alpha1(III) chains; type III collagen triple helices associate to form fibrils. Relationships: is a type of fibrillar collagen trimer [GO:0005583]